bundle sheath cell differentiation [GO:1903498] (biological process) References: PMID:24517883 Sources: GOC:TermGenie, GOC:tb, GO_REF:0000086 Definition: The process in which a relatively unspecialized cell acquires the specialized features of a bundle sheath cell. Relationships: is a type of GO:0030154